{
  "gene_name": "Unconventional myosin-VI",
  "gene_symbol": "MYO6",
  "gene": "UniProtKB:Q9UM54",
  "term_label": "endocytosis",
  "term_id": "GO:0006897"
}